Mo-molybdopterin cofactor biosynthetic process [GO:0006777] (biological process) References: PMID:22370186, PMID:23201473 Sources: ISSN:09498257 Also known as: Mo-molybdopterin cofactor anabolism, Mo-molybdopterin cofactor biosynthesis, Mo-molybdopterin cofactor formation, Mo-molybdopterin cofactor synthesis, Moco biosynthesis, Moco biosynthetic process, molybdenum cofactor biosynthetic process Subtypes: bis(molybdopterin guanine dinucleotide)molybdenum biosynthetic process [GO:1902758], GO:1902760 Relationships: is a type of GO:0019720; is a type of molybdopterin cofactor biosynthetic process [GO:0032324]; has part molybdenum incorporation into molybdenum-molybdopterin complex [GO:0018315]; has part GTP 3',8'-cyclase activity [GO:0061798]; BFO_0000051 GO:0061799 Definition: The chemical reactions and pathways resulting in the formation of the Mo-molybdopterin cofactor, essential for the catalytic activity of some enzymes. The cofactor consists of a mononuclear molybdenum (Mo) ion coordinated by one or two molybdopterin ligands.